{
  "gene": "UniProtKB:Q9BRG2",
  "gene_symbol": "SH2D3A",
  "term_id": "UNKNOWN:0001",
  "term_label": "Unknown molecular function",
  "gene_name": "SH2 domain-containing protein 3A"
}